{
  "gene": "UniProtKB:Q86WI1",
  "gene_symbol": "PKHD1L1",
  "term_label": "Unknown biological process",
  "term_id": "UNKNOWN:0002",
  "gene_name": "Fibrocystin-L"
}